{
  "term_label": "Unknown cellular component",
  "term_id": "UNKNOWN:0003",
  "gene": "UniProtKB:P0C7N1",
  "gene_name": "Olfactory receptor 8U8",
  "gene_symbol": "OR8U8"
}